{
  "gene_name": "Glucose-fructose oxidoreductase domain-containing protein 2",
  "gene": "UniProtKB:Q3B7J2",
  "term_label": "extracellular matrix",
  "gene_symbol": "GFOD2",
  "term_id": "GO:0031012"
}